establishment of meiotic spindle localization [GO:0051295] (biological process) Subtypes: establishment of meiotic spindle orientation [GO:0051296] Sources: GOC:ai Definition: The cell cycle process in which the directed movement of the meiotic spindle to a specific location in the cell occurs. Also known as: establishment of meiotic spindle localisation, meiotic spindle positioning, spindle positioning involved in meiotic cell cycle, spindle positioning during meiosis Relationships: is a type of establishment of spindle localization [GO:0051293]; is a type of GO:1903046